{
  "gene": "UniProtKB:P83369",
  "gene_name": "U7 snRNA-associated Sm-like protein LSm11",
  "term_label": "U7 snRNA binding",
  "gene_symbol": "LSM11",
  "term_id": "GO:0071209"
}